{
  "term_label": "RNA polymerase II cis-regulatory region sequence-specific DNA binding",
  "term_id": "GO:0000978",
  "gene_name": "Zinc finger protein Gfi-1",
  "gene_symbol": "GFI1",
  "gene": "UniProtKB:Q99684"
}